premature acrosome loss [GO:0061948] (biological process) Relationships: is a type of reproductive process [GO:0022414] Note: If the release of the acrosome content when the sperm reaches to the zona pellucida, consider using acrosome reaction. Also known as: spontaneous acrosome loss Definition: The discharge, by sperm, of a single, anterior secretory granule before the sperm reaches to the zona pellucida of the oocyte. The process begins with the fusion of the outer acrosomal membrane with the sperm plasma membrane and ends with the exocytosis of the acrosomal contents. References: PMID:19153666, PMID:21380641, PMID:26655718 Regulation: regulated by GO:0061949; negatively regulated by negative regulation of premature acrosome loss [GO:0061950]